{
  "gene_name": "Oxysterol-binding protein-related protein 8",
  "term_label": "membrane",
  "term_id": "GO:0016020",
  "gene": "UniProtKB:Q9BZF1",
  "gene_symbol": "OSBPL8"
}